{
  "term_label": "cytosol",
  "term_id": "GO:0005829",
  "gene_name": "Adenylosuccinate lyase",
  "gene": "UniProtKB:P30566",
  "gene_symbol": "ADSL"
}